{
  "gene": "UniProtKB:Q76B58",
  "gene_name": "BMP_retinoic acid-inducible neural-specific protein 3",
  "term_id": "GO:0005737",
  "gene_symbol": "BRINP3",
  "term_label": "cytoplasm"
}